negative regulation of methane biosynthetic process from trimethylamine [GO:1900331] (BP) Definition: Any process that stops, prevents or reduces the frequency, rate or extent of methane biosynthetic process from trimethylamine. Also known as: down regulation of methane biosynthetic process from trimethylamine, down-regulation of methane biosynthetic process from trimethylamine, downregulation of methane biosynthetic process from trimethylamine, inhibition of methane biosynthetic process from trimethylamine Relationships: is a type of negative regulation of amine metabolic process [GO:0033239]; is a type of GO:1900330; is a type of negative regulation of alkane biosynthetic process [GO:1901578]; is_a negative regulation of cellular respiration [GO:1901856]; negatively regulates methane biosynthetic process from trimethylamine [GO:2001130] Sources: GOC:TermGenie, GOC:mengo_curators